{
  "term_label": "four-way junction helicase activity",
  "term_id": "GO:0009378",
  "gene": "UniProtKB:O94761",
  "gene_symbol": "RECQL4",
  "gene_name": "ATP-dependent DNA helicase Q4"
}